{
  "gene_symbol": "B3GNT8",
  "gene": "UniProtKB:Q7Z7M8",
  "term_label": "protein N-acetylglucosaminyltransferase activity",
  "term_id": "GO:0016262",
  "gene_name": "UDP-GlcNAc:betaGal beta-1,3-N-acetylglucosaminyltransferase 8"
}